{
  "gene": "UniProtKB:O95257",
  "gene_name": "Growth arrest and DNA damage-inducible protein GADD45 gamma",
  "term_label": "regulation of cell cycle",
  "term_id": "GO:0051726",
  "gene_symbol": "GADD45G"
}